{
  "gene_name": "TLC domain-containing protein 4",
  "gene": "UniProtKB:Q96MV1",
  "term_label": "Unknown molecular function",
  "term_id": "UNKNOWN:0001",
  "gene_symbol": "TLCD4"
}